{
  "gene": "UniProtKB:Q9H7J1",
  "gene_symbol": "PPP1R3E",
  "term_id": "GO:0005979",
  "gene_name": "Protein phosphatase 1 regulatory subunit 3E",
  "term_label": "regulation of glycogen biosynthetic process"
}